{
  "gene": "UniProtKB:O43316",
  "gene_name": "Paired box protein Pax-4",
  "term_id": "GO:0003309",
  "term_label": "type B pancreatic cell differentiation",
  "gene_symbol": "PAX4"
}